regulation of connective tissue replacement [GO:1905203] (biological process) Relationships: is a type of GO:0034103; RO_0002211 connective tissue replacement [GO:0097709] Definition: Any process that modulates the frequency, rate or extent of connective tissue replacement. References: PMID:25590961 Sources: GOC:BHF, GOC:BHF_miRNA, GOC:TermGenie, GOC:bc, GO_REF:0000058 Subtypes: regulation of connective tissue replacement involved in inflammatory response wound healing [GO:1904596], negative regulation of connective tissue replacement [GO:1905204], positive regulation of connective tissue replacement [GO:1905205]